negative regulation of fatty acid transport [GO:2000192] (biological process) Relationships: is a type of negative regulation of lipid transport [GO:0032369]; is a type of negative regulation of organic acid transport [GO:0032891]; is a type of GO:2000191; negatively regulates fatty acid transport [GO:0015908] Definition: Any process that stops, prevents, or reduces the frequency, rate or extent of fatty acid transport. Sources: GOC:BHF Subtypes: GO:0032304, negative regulation of long-chain fatty acid import into cell [GO:0140213]